{
  "gene_name": "Immunoglobulin alpha Fc receptor",
  "term_id": "GO:0002767",
  "term_label": "immune response-inhibiting cell surface receptor signaling pathway",
  "gene": "UniProtKB:P24071",
  "gene_symbol": "FCAR"
}